Skp1-protein-hydroxyproline N-acetylglucosaminyltransferase activity [GO:0033830] (molecular function) Definition: Catalysis of the reaction: UDP-N-acetylglucosamine + Skp1-protein-hydroxyproline = UDP + Skp1-protein-O-(N-acetyl-D-glucosaminyl)hydroxyproline. Also known as: Skp1-HyPro GlcNAc-transferase activity, UDP-GlcNAc:Skp1-hydroxyproline GlcNAc-transferase activity, UDP-GlcNAc:hydroxyproline polypeptide GlcNAc-transferase activity, UDP-N-acetyl-D-glucosamine:Skp1-protein-hydroxyproline N-acetyl-D-glucosaminyl-transferase activity, UDP-N-acetylglucosamine (GlcNAc):hydroxyproline polypeptide GlcNAc-transferase activity Sources: EC:2.4.1.229 Relationships: is a type of acetylglucosaminyltransferase activity [GO:0008375]; is a type of GO:0140096